{
  "gene_name": "Mitogen-activated protein kinase kinase kinase kinase 5",
  "gene": "UniProtKB:Q9Y4K4",
  "gene_symbol": "MAP4K5",
  "term_id": "GO:0005737",
  "term_label": "cytoplasm"
}